{
  "gene_name": "26S proteasome non-ATPase regulatory subunit 2",
  "term_id": "GO:0034515",
  "gene": "UniProtKB:Q13200",
  "gene_symbol": "PSMD2",
  "term_label": "proteasome storage granule"
}